{
  "gene": "UniProtKB:Q9NY93",
  "term_id": "UNKNOWN:0001",
  "gene_name": "Probable ATP-dependent RNA helicase DDX56",
  "term_label": "Unknown molecular function",
  "gene_symbol": "DDX56"
}